{
  "term_id": "GO:1990726",
  "gene_symbol": "LSM7",
  "term_label": "Lsm1-7-Pat1 complex",
  "gene_name": "U6 snRNA-associated Sm-like protein LSm7",
  "gene": "UniProtKB:Q9UK45"
}